{
  "gene_symbol": "RP2",
  "term_id": "GO:0005929",
  "gene_name": "Protein XRP2",
  "gene": "UniProtKB:O75695",
  "term_label": "cilium"
}